{
  "term_id": "GO:0005615",
  "term_label": "extracellular space",
  "gene_name": "Tubulointerstitial nephritis antigen-like",
  "gene": "UniProtKB:Q9GZM7",
  "gene_symbol": "TINAGL1"
}